{
  "term_label": "Unknown molecular function",
  "gene_name": "Golgi-associated RAB2 interactor protein 3",
  "gene": "UniProtKB:Q8TC56",
  "gene_symbol": "GARIN3",
  "term_id": "UNKNOWN:0001"
}